{
  "term_id": "GO:0004722",
  "gene": "UniProtKB:O14830",
  "gene_symbol": "PPEF2",
  "gene_name": "Serine_threonine-protein phosphatase with EF-hands 2",
  "term_label": "protein serine/threonine phosphatase activity"
}